{
  "gene_symbol": "LAMB4",
  "gene": "UniProtKB:A4D0S4",
  "gene_name": "Laminin subunit beta-4",
  "term_label": "extracellular space",
  "term_id": "GO:0005615"
}